{
  "gene_name": "Sodium channel and clathrin linker 1",
  "term_label": "centriole",
  "gene": "UniProtKB:Q96NL6",
  "gene_symbol": "SCLT1",
  "term_id": "GO:0005814"
}